{
  "term_label": "actin filament network formation",
  "term_id": "GO:0051639",
  "gene": "UniProtKB:P13796",
  "gene_symbol": "LCP1",
  "gene_name": "Plastin-2"
}